{
  "term_id": "GO:0005634",
  "gene_name": "Transcription factor SOX-1",
  "term_label": "nucleus",
  "gene": "UniProtKB:O00570",
  "gene_symbol": "SOX1"
}